{
  "gene_symbol": "RAB20",
  "gene_name": "Ras-related protein Rab-20",
  "gene": "UniProtKB:Q9NX57",
  "term_label": "intracellular protein transport",
  "term_id": "GO:0006886"
}